{
  "term_id": "GO:0006887",
  "gene_name": "Synaptotagmin-like protein 2",
  "gene": "UniProtKB:Q9HCH5",
  "term_label": "exocytosis",
  "gene_symbol": "SYTL2"
}